{
  "term_id": "UNKNOWN:0001",
  "gene_name": "Putative uncharacterized protein encoded by LINC01559",
  "gene_symbol": "LINC01559",
  "gene": "UniProtKB:Q495D7",
  "term_label": "Unknown molecular function"
}